{
  "term_id": "GO:0006955",
  "gene": "UniProtKB:A0A075B6S6",
  "gene_symbol": "IGKV2D-30",
  "term_label": "immune response",
  "gene_name": "Immunoglobulin kappa variable 2D-30"
}